{
  "term_label": "nucleus",
  "gene": "UniProtKB:P07199",
  "gene_symbol": "CENPB",
  "gene_name": "Major centromere autoantigen B",
  "term_id": "GO:0005634"
}